{
  "term_id": "GO:0003690",
  "gene_name": "Interferon-inducible protein AIM2",
  "gene": "UniProtKB:O14862",
  "term_label": "double-stranded DNA binding",
  "gene_symbol": "AIM2"
}